PR-DUB complex [GO:0035517] (cellular component) Relationships: is_a GO:0031519 Definition: A multimeric protein complex that removes monoubiquitin from histone H2A. In Drosophila and mammals, the core of the complex is composed of Calypso/BAP1 and Asx/ASXL1, respectively. References: PMID:20436459 Also known as: Polycomb repressive deubiquitinase complex